{
  "term_label": "Unknown molecular function",
  "term_id": "UNKNOWN:0001",
  "gene_symbol": "CFAP300",
  "gene": "UniProtKB:Q9BRQ4",
  "gene_name": "Cilia- and flagella-associated protein 300"
}